{
  "term_label": "lysosome",
  "gene": "UniProtKB:Q9NXL6",
  "gene_symbol": "SIDT1",
  "gene_name": "SID1 transmembrane family member 1",
  "term_id": "GO:0005764"
}